{
  "term_id": "UNKNOWN:0002",
  "term_label": "Unknown biological process",
  "gene_symbol": "OSCP1",
  "gene": "UniProtKB:Q8WVF1",
  "gene_name": "Protein OSCP1"
}